positive regulation of TRAIL production [GO:0032759] (biological process) Definition: Any process that activates or increases the frequency, rate, or extent of TRAIL production. Sources: GOC:mah Relationships: is a type of regulation of TRAIL production [GO:0032679]; is a type of positive regulation of tumor necrosis factor superfamily cytokine production [GO:1903557]; positively regulates GO:0032639 Also known as: up regulation of TRAIL production, up-regulation of TRAIL production, upregulation of TRAIL production, activation of TRAIL production, positive regulation of TRAIL biosynthetic process, stimulation of TRAIL production